propionate biosynthetic process [GO:0019542] (BP) Also known as: propionate anabolism, propionate biosynthesis, propionate formation, propionate synthesis Relationships: is a type of GO:0019541; is a type of short-chain fatty acid biosynthetic process [GO:0051790] Sources: GOC:go_curators Definition: The chemical reactions and pathways resulting in the formation of propionate, the anion derived from propionic acid.